mannosylglycoprotein endo-beta-mannosidase activity [GO:0033947] (molecular function) Definition: Catalysis of the hydrolysis of the alpha-D-mannosyl-(1->6)-beta-D-mannosyl-(1->4)-beta-D-N-acetylglucosaminyl-(1->4)-beta-D-N-acetylglucosaminyl sequence of glycoprotein to alpha-D-mannosyl-(1->6)-D-mannose and beta-D-N-acetylglucosaminyl-(1->4)-beta-D-N-acetylglucosaminyl sequences. Relationships: is a type of beta-mannosidase activity [GO:0004567] Also known as: endo-beta-mannosidase activity Sources: EC:3.2.1.152